{
  "gene_name": "Anoctamin-7",
  "term_id": "GO:0061588",
  "gene": "UniProtKB:Q6IWH7",
  "gene_symbol": "ANO7",
  "term_label": "calcium activated phospholipid scrambling"
}